regulation of sphingolipid mediated signaling pathway [GO:1902068] (biological process) Subtypes: negative regulation of sphingolipid mediated signaling pathway [GO:1902069], positive regulation of sphingolipid mediated signaling pathway [GO:1902070] Relationships: is a type of regulation of signal transduction [GO:0009966]; regulates sphingolipid mediated signaling pathway [GO:0090520] Definition: Any process that modulates the frequency, rate or extent of sphingolipid signaling. Also known as: regulation of sphingolipid signaling pathway References: PMID:20870412 Sources: GOC:TermGenie